{
  "term_id": "GO:0005737",
  "term_label": "cytoplasm",
  "gene_symbol": "TRIM61",
  "gene": "UniProtKB:Q5EBN2",
  "gene_name": "Putative tripartite motif-containing protein 61"
}